{
  "term_label": "eosinophil chemotaxis",
  "gene_name": "C-C motif chemokine 24",
  "gene_symbol": "CCL24",
  "gene": "UniProtKB:O00175",
  "term_id": "GO:0048245"
}